{
  "gene_symbol": "UGT1A1",
  "term_label": "estrogen metabolic process",
  "gene": "UniProtKB:P22309",
  "term_id": "GO:0008210",
  "gene_name": "UDP-glucuronosyltransferase 1A1"
}